spore wall biogenesis [GO:0070590] (biological process) Relationships: is a type of GO:0042546; is part of GO:0030435 Subtypes: ascospore wall biogenesis [GO:0070591] Sources: GOC:mah Definition: A cellular process that results in the biosynthesis of constituent macromolecules, assembly, and arrangement of constituent parts of a spore wall. A spore wall is the specialized cell wall lying outside the cell membrane of a spore.